{
  "term_label": "mRNA 3'-end processing by stem-loop binding and cleavage",
  "term_id": "GO:0006398",
  "gene": "UniProtKB:Q9P2I0",
  "gene_symbol": "CPSF2",
  "gene_name": "Cleavage and polyadenylation specificity factor subunit 2"
}